{
  "gene_symbol": "MBTPS1",
  "term_id": "GO:0004252",
  "term_label": "serine-type endopeptidase activity",
  "gene": "UniProtKB:Q14703",
  "gene_name": "Membrane-bound transcription factor site-1 protease"
}